polyamine import across plasma membrane [GO:0140202] (BP) Relationships: is a type of nitrogen compound transport [GO:0071705]; is a type of import across plasma membrane [GO:0098739] Subtypes: spermidine import across plasma membrane [GO:0140203] Definition: The directed movement of a polyamine from outside of a cell, across the plasma membrane and into the cytosol. References: PMID:17218313